{
  "gene_name": "Zinc finger protein 273",
  "gene": "UniProtKB:Q14593",
  "term_label": "RNA polymerase II cis-regulatory region sequence-specific DNA binding",
  "term_id": "GO:0000978",
  "gene_symbol": "ZNF273"
}